{
  "gene_symbol": "OR5I1",
  "term_id": "UNKNOWN:0003",
  "gene_name": "Olfactory receptor 5I1",
  "term_label": "Unknown cellular component",
  "gene": "UniProtKB:Q13606"
}